{
  "gene_name": "TBC1 domain family member 22B",
  "term_id": "GO:0005794",
  "term_label": "Golgi apparatus",
  "gene_symbol": "TBC1D22B",
  "gene": "UniProtKB:Q9NU19"
}